{
  "gene_name": "Cyclin-dependent kinase inhibitor 3",
  "gene_symbol": "CDKN3",
  "term_label": "Unknown biological process",
  "term_id": "UNKNOWN:0002",
  "gene": "UniProtKB:Q16667"
}